{
  "term_label": "Unknown molecular function",
  "gene": "UniProtKB:Q9UJQ7",
  "gene_name": "SCP2 sterol-binding domain-containing protein 1",
  "term_id": "UNKNOWN:0001",
  "gene_symbol": "SCP2D1"
}